{
  "term_label": "signal transduction",
  "gene_symbol": "GAB1",
  "gene": "UniProtKB:Q13480",
  "term_id": "GO:0007165",
  "gene_name": "GRB2-associated-binding protein 1"
}